{
  "term_id": "GO:0043122",
  "gene": "UniProtKB:Q99829",
  "gene_name": "Copine-1",
  "term_label": "regulation of canonical NF-kappaB signal transduction",
  "gene_symbol": "CPNE1"
}